phosphatidylinositol bisphosphate binding [GO:1902936] (molecular function) Relationships: is a type of phosphatidylinositol phosphate binding [GO:1901981] Subtypes: phosphatidylinositol-4,5-bisphosphate binding [GO:0005546], GO:0080025 References: PMID:18690034 Sources: GOC:TermGenie, GOC:bhm, GO_REF:0000067 Note: An example of this is KCNJ2 in human (P63252) in PMID:18690034 (inferred from direct assay) Definition: Binding to phosphatidylinositol bisphosphate.